negative regulation of chloroplast fission [GO:1905193] (biological process) Definition: Any process that stops, prevents or reduces the frequency, rate or extent of chloroplast fission. Note: Any process that modulates the rate, frequency or extent of chloroplast fission. Chloroplast fission is the division of a chloroplast within a cell to form two or more separate chloroplast compartments. Also known as: down regulation of chloroplast division, down regulation of chloroplast fission, down-regulation of chloroplast division, down-regulation of chloroplast fission, downregulation of chloroplast division, downregulation of chloroplast fission, negative regulation of chloroplast division, inhibition of chloroplast division, inhibition of chloroplast fission Relationships: is a type of negative regulation of organelle organization [GO:0010639]; is a type of regulation of chloroplast fission [GO:1905192]; negatively regulates chloroplast fission [GO:0010020] References: PMID:26862170 Sources: GOC:TermGenie, GO_REF:0000058